{
  "term_label": "fibroblast growth factor receptor signaling pathway",
  "term_id": "GO:0008543",
  "gene": "UniProtKB:O43559",
  "gene_name": "Fibroblast growth factor receptor substrate 3",
  "gene_symbol": "FRS3"
}